{
  "gene": "UniProtKB:Q8IVB4",
  "gene_symbol": "SLC9A9",
  "term_label": "sodium ion import across plasma membrane",
  "term_id": "GO:0098719",
  "gene_name": "Sodium_hydrogen exchanger 9"
}